{
  "term_id": "UNKNOWN:0002",
  "gene": "UniProtKB:P18089",
  "gene_name": "Alpha-2B adrenergic receptor",
  "gene_symbol": "ADRA2B",
  "term_label": "Unknown biological process"
}